{
  "term_id": "GO:0005737",
  "gene_symbol": "SPATA33",
  "gene_name": "Spermatogenesis-associated protein 33",
  "term_label": "cytoplasm",
  "gene": "UniProtKB:Q96N06"
}